{
  "gene_name": "Leucine-rich repeat and immunoglobulin-like domain-containing nogo receptor-interacting protein 1",
  "term_label": "neuron development",
  "gene": "UniProtKB:Q96FE5",
  "gene_symbol": "LINGO1",
  "term_id": "GO:0048666"
}